cortical dynamic polarity patch [GO:0090726] (cellular component) References: PMID:23200991 Sources: GOC:mah Also known as: dynamic polarity patch at the cell cortex Relationships: is a type of cellular anatomical structure [GO:0110165]; is part of GO:0005938 Definition: A region of the cell cortex that contains a higher concentration of growth polarity factors than the surrounding cortex and that changes position over time. An example is found in fission yeast cells during early mating, in which the GTPase Cdc42 dynamically to discrete zones within the cortex prior to shmoo formation.